{
  "gene_symbol": "CROCCP3",
  "gene": "UniProtKB:Q8IVE0",
  "term_label": "Unknown cellular component",
  "gene_name": "Putative ciliary rootlet coiled-coil protein-like 2 protein",
  "term_id": "UNKNOWN:0003"
}